{
  "term_id": "UNKNOWN:0003",
  "term_label": "Unknown cellular component",
  "gene_name": "Keratin-associated protein 22-2",
  "gene_symbol": "KRTAP22-2",
  "gene": "UniProtKB:Q3LI68"
}